{
  "term_label": "action potential",
  "gene_name": "Potassium voltage-gated channel subfamily C member 3",
  "gene": "UniProtKB:Q14003",
  "term_id": "GO:0001508",
  "gene_symbol": "KCNC3"
}